{
  "term_id": "GO:0005666",
  "gene_symbol": "POLR3C",
  "gene": "UniProtKB:Q9BUI4",
  "term_label": "RNA polymerase III complex",
  "gene_name": "DNA-directed RNA polymerase III subunit RPC3"
}